juvenile hormone secretion [GO:0045443] (biological process) Regulation: regulated by regulation of juvenile hormone secretion [GO:0007558]; negatively regulated by GO:0045972; positively regulated by positive regulation of juvenile hormone secretion [GO:0045973] Relationships: is a type of GO:0046865; is a type of endocrine hormone secretion [GO:0060986]; is a type of lipid export from cell [GO:0140353] Definition: The regulated release of juvenile hormones, the three sesquiterpenoid derivatives that function to maintain the larval state of insects at molting and that may be required for other processes, e.g. oogenesis. Sources: GOC:go_curators, ISBN:0198547684